{
  "gene": "UniProtKB:Q9NY43",
  "term_id": "GO:0005634",
  "term_label": "nucleus",
  "gene_name": "BarH-like 2 homeobox protein",
  "gene_symbol": "BARHL2"
}